{
  "term_label": "nucleoplasm",
  "gene_name": "Serine_threonine_tyrosine-interacting protein",
  "gene": "UniProtKB:Q8WUJ0",
  "term_id": "GO:0005654",
  "gene_symbol": "STYX"
}